left anterior flagellum [GO:0097554] (cellular component) References: PMID:16607022, PMID:5961344 Sources: GOC:giardia, ISBN:9780124260207 Definition: A cilium (also called flagellum) found in Giardia species (trophozoite stage). It originates at the left anterior basal body, extends laterally through the cytoplasm, crosses the right anterior axoneme, and exits as a membrane-bound flagellum on the anterior left side of the cell. Also known as: left anterior cilium Relationships: is a type of 9+2 motile cilium [GO:0097729] Note: Note that we deem cilium and microtubule-based flagellum to be equivalent; the primary term name reflects frequency of use. Also note that, due to the asymmetric nature of the Giardia trophozoite, this term is defined spatially as the trophozoite is viewed from the dorsal side, with the two nuclei dorsal to the ventral disc, and the ventral disc toward the anterior.